{
  "term_label": "intraciliary transport",
  "gene_symbol": "IFT46",
  "term_id": "GO:0042073",
  "gene_name": "Intraflagellar transport protein 46 homolog",
  "gene": "UniProtKB:Q9NQC8"
}